{
  "gene_symbol": "C14orf119",
  "term_label": "Unknown biological process",
  "gene": "UniProtKB:Q9NWQ9",
  "term_id": "UNKNOWN:0002",
  "gene_name": "Uncharacterized protein C14orf119"
}